chromate transmembrane transporter activity [GO:0015109] (molecular function) Sources: GOC:ai Definition: Enables the transfer of chromate from one side of a membrane to the other. Chromate is the anion of chromic acid, H2CrO4 (aq) or CrO3. Relationships: is a type of GO:0022857; is part of chromate transport [GO:0015703]